{
  "gene": "UniProtKB:Q8IV48",
  "gene_name": "3'-5' exoribonuclease 1",
  "term_id": "GO:0005730",
  "gene_symbol": "ERI1",
  "term_label": "nucleolus"
}